{
  "term_id": "GO:0006955",
  "gene_symbol": "IGLV3-32",
  "gene": "UniProtKB:A0A0A0MS00",
  "gene_name": "Probable non-functional immunoglobulin lambda variable 3-32",
  "term_label": "immune response"
}